cellular birth scar [GO:0071597] (CC) References: PMID:16672383, PMID:7730409 Sources: GOC:mcc Definition: Crater-like ring of chitinous scar tissue located on the surface of the daughter cell, in budding fungi, at the site of separation from the mother cell. It is formed after the newly emerged daughter cell separates, thereby marking the site of cytokinesis and septation. Relationships: is a type of cellular anatomical structure [GO:0110165]; is part of fungal-type cell wall [GO:0009277]